{
  "gene_name": "General transcription factor 3C polypeptide 6",
  "gene": "UniProtKB:Q969F1",
  "term_id": "UNKNOWN:0001",
  "term_label": "Unknown molecular function",
  "gene_symbol": "GTF3C6"
}